signal peptidase complex [GO:0005787] (cellular component) Definition: A protein complex that is located in the endoplasmic reticulum membrane and cleaves the signal sequence from precursor proteins following their transport out of the cytoplasmic space. References: PMID:1846444, PMID:7615509 Sources: GOC:sgd_curators Relationships: is a type of membrane protein complex [GO:0098796]; is a type of GO:0140534; is a type of serine-type endopeptidase complex [GO:1905370]; is part of endoplasmic reticulum membrane [GO:0005789]